optic chiasma development [GO:0061360] (biological process) Definition: The developmental process pertaining to the progression of the optic chiasm from its initial formation to the mature structure. The process begins when the pathfinding of the axons of the developing optic nerve cause some axons to cross at the midline of the brain and ends when the axons are mature. Sources: GOC:dph Relationships: is a type of anatomical structure development [GO:0048856]; is part of optic nerve development [GO:0021554] Also known as: optic chiasm development